{
  "term_id": "GO:0007608",
  "gene_symbol": "OR9Q2",
  "term_label": "sensory perception of smell",
  "gene_name": "Olfactory receptor 9Q2",
  "gene": "UniProtKB:Q8NGE9"
}